intracellularly ATP-gated chloride channel activity [GO:0005260] (molecular function) Also known as: CFTR, cystic fibrosis transmembrane conductance regulator, channel-conductance-controlling ATPase activity Relationships: is a type of chloride channel activity [GO:0005254]; is a type of ligand-gated monoatomic anion channel activity [GO:0099095]; is a type of intracellularly ATP-gated ion channel activity [GO:0099142]; is a type of polypeptide conformation or assembly isomerase activity [GO:0120544] Note: This activity is a phosphorylation and ATP-gated anion channel, increasing the conductance for certain anions (e.g. Cl-) to flow down their electrochemical gradient. ATP-driven conformational changes in CFTR open and close a gate to allow transmembrane flow of anions down their electrochemical gradient.This in contrast to other ABC proteins, in which ATP-driven conformational changes fuel uphill substrate transport across cellular membranes. Essentially, CFTR is an ion channel that evolved as a 'broken' ABC transporter that leaks when in open conformation (from Wikipedia:Cystic_fibrosis_transmembrane_conductance_regulator). Definition: Enables passage of a chloride ion through a transmembrane channel that opens when ATP is bound by the channel complex or one of its constituent parts on the intracellular side of the plasma membrane. References: PMID:24727426, PMID:9922375